{
  "gene_name": "Rho-related GTP-binding protein RhoG",
  "term_id": "GO:0016601",
  "term_label": "Rac protein signal transduction",
  "gene_symbol": "RHOG",
  "gene": "UniProtKB:P84095"
}